{
  "term_id": "GO:0005634",
  "gene": "UniProtKB:Q9H967",
  "term_label": "nucleus",
  "gene_name": "WD repeat-containing protein 76",
  "gene_symbol": "WDR76"
}